{
  "gene_name": "Olfactory receptor 8D1",
  "term_id": "GO:0005549",
  "gene_symbol": "OR8D1",
  "term_label": "odorant binding",
  "gene": "UniProtKB:Q8WZ84"
}